{
  "term_id": "GO:0019367",
  "term_label": "fatty acid elongation, saturated fatty acid",
  "gene_symbol": "ELOVL4",
  "gene_name": "Elongation of very long chain fatty acids protein 4",
  "gene": "UniProtKB:Q9GZR5"
}